acetylcholine-gated monoatomic cation-selective channel activity [GO:0022848] (MF) Relationships: is a type of excitatory extracellular ligand-gated monoatomic ion channel activity [GO:0005231]; is a type of ligand-gated monoatomic cation channel activity [GO:0099094]; is a type of transmitter-gated monoatomic ion channel activity involved in regulation of postsynaptic membrane potential [GO:1904315] Definition: Selectively enables the transmembrane transfer of a cation by a channel that opens upon binding acetylcholine. Also known as: acetylcholine-gated cation-selective channel activity, acetylcholine-activated cation-selective channel activity, acetylcholine-gated cation channel activity, ionotropic acetylcholine receptor activity, nAChR, nicotinergic acetylcholine receptor activity, nicotinic acetylcholine-activated cation-selective channel activity References: PMID:2466967 Sources: GOC:mah